{
  "gene_symbol": "SMAD9",
  "gene_name": "Mothers against decapentaplegic homolog 9",
  "gene": "UniProtKB:O15198",
  "term_label": "anatomical structure morphogenesis",
  "term_id": "GO:0009653"
}